locus ceruleus development [GO:0021703] (biological process) Sources: GOC:cls, GOC:dgh, GOC:dph, GOC:jid, GO_REF:0000021 Relationships: is a type of neural nucleus development [GO:0048857]; is part of pons development [GO:0021548] Definition: The process whose specific outcome is the progression of the locus ceruleus over time, from its formation to the mature structure. The locus ceruleus is a dense cluster of neurons within the dorsorostral pons. This nucleus is the major location of neurons that release norepinephrine throughout the brain, and is responsible for physiological responses to stress and panic. Also known as: locus caeruleus development, locus coeruleus development